{
  "term_id": "UNKNOWN:0003",
  "gene_name": "Olfactory receptor 5K4",
  "term_label": "Unknown cellular component",
  "gene": "UniProtKB:A6NMS3",
  "gene_symbol": "OR5K4"
}